negative regulation of austinol biosynthetic process [GO:1900641] (biological process) Also known as: down regulation of austinol anabolism, down regulation of austinol biosynthesis, down regulation of austinol biosynthetic process, down regulation of austinol formation, down regulation of austinol synthesis, down-regulation of austinol anabolism, down-regulation of austinol biosynthesis, down-regulation of austinol biosynthetic process, down-regulation of austinol formation, down-regulation of austinol synthesis, downregulation of austinol anabolism, downregulation of austinol biosynthesis, downregulation of austinol biosynthetic process, downregulation of austinol formation, downregulation of austinol synthesis, inhibition of austinol anabolism, inhibition of austinol biosynthesis, inhibition of austinol formation, inhibition of austinol synthesis, negative regulation of austinol anabolism, negative regulation of austinol biosynthesis, negative regulation of austinol formation, negative regulation of austinol synthesis, inhibition of austinol biosynthetic process Definition: Any process that stops, prevents or reduces the frequency, rate or extent of austinol biosynthetic process. Sources: GOC:TermGenie, GOC:di Relationships: is_a negative regulation of biosynthetic process [GO:0009890]; is a type of regulation of austinol biosynthetic process [GO:1900640]; RO_0002212 austinol biosynthetic process [GO:1900560]